{
  "term_label": "cell-cell junction assembly",
  "term_id": "GO:0007043",
  "gene_name": "Cadherin-19",
  "gene_symbol": "CDH19",
  "gene": "UniProtKB:Q9H159"
}